{
  "gene_name": "Stonin-1",
  "gene": "UniProtKB:Q9Y6Q2",
  "term_label": "AP-1 adaptor complex",
  "gene_symbol": "STON1",
  "term_id": "GO:0030121"
}